urease activator complex [GO:0150006] (cellular component) Relationships: is a type of enzyme activator complex [GO:0150005] Definition: A protein complex required for the activation of urease. Activator subunits dissociate before urease has catalytic function. References: PMID:16244137, PMID:28710280 Sources: GOC:bhm